{
  "term_label": "Unknown biological process",
  "gene_name": "Coiled-coil domain-containing protein 190",
  "gene": "UniProtKB:Q86UF4",
  "gene_symbol": "CCDC190",
  "term_id": "UNKNOWN:0002"
}